{
  "gene_symbol": "ABL1",
  "gene_name": "Tyrosine-protein kinase ABL1",
  "term_label": "plasma membrane",
  "gene": "UniProtKB:P00519",
  "term_id": "GO:0005886"
}